{
  "gene_name": "Ryanodine receptor 2",
  "term_label": "smooth endoplasmic reticulum",
  "term_id": "GO:0005790",
  "gene_symbol": "RYR2",
  "gene": "UniProtKB:Q92736"
}